{
  "gene_symbol": "STX17",
  "term_id": "GO:0012505",
  "gene": "UniProtKB:P56962",
  "gene_name": "Syntaxin-17",
  "term_label": "endomembrane system"
}